negative regulation of phenotypic switching [GO:1900240] (biological process) Sources: GOC:TermGenie, GOC:di Also known as: down regulation of phenotypic switching, down-regulation of phenotypic switching, downregulation of phenotypic switching, inhibition of phenotypic switching, down regulation of phenotypic dimorphism, down-regulation of phenotypic dimorphism, downregulation of phenotypic dimorphism, inhibition of phenotypic dimorphism, negative regulation of phenotypic dimorphism Relationships: is a type of negative regulation of cellular process [GO:0048523]; is a type of regulation of phenotypic switching [GO:1900239]; negatively regulates phenotypic switching [GO:0036166] Definition: Any process that stops, prevents or reduces the frequency, rate or extent of phenotypic switching. Subtypes: negative regulation of cell differentiation involved in phenotypic switching [GO:1905916]